{
  "term_id": "GO:0032982",
  "gene_name": "Unconventional myosin-XVIIIb",
  "term_label": "myosin filament",
  "gene": "UniProtKB:Q8IUG5",
  "gene_symbol": "MYO18B"
}